{
  "gene_symbol": "TRIM56",
  "term_id": "GO:0060340",
  "gene": "UniProtKB:Q9BRZ2",
  "term_label": "positive regulation of type I interferon-mediated signaling pathway",
  "gene_name": "E3 ubiquitin-protein ligase TRIM56"
}